{
  "term_id": "GO:0008420",
  "gene_symbol": "SSU72L5",
  "term_label": "RNA polymerase II CTD heptapeptide repeat phosphatase activity",
  "gene": "UniProtKB:A0A1W2PQ64",
  "gene_name": "RNA polymerase II subunit A C-terminal domain phosphatase SSU72 like protein 5"
}